{
  "term_id": "GO:0042178",
  "gene_symbol": "CYP2C9",
  "term_label": "xenobiotic catabolic process",
  "gene": "UniProtKB:P11712",
  "gene_name": "Cytochrome P450 2C9"
}